{
  "gene": "UniProtKB:Q8IXB1",
  "term_label": "endoplasmic reticulum lumen",
  "gene_symbol": "DNAJC10",
  "gene_name": "DnaJ homolog subfamily C member 10",
  "term_id": "GO:0005788"
}